{
  "gene_symbol": "OR2G3",
  "term_id": "GO:0050911",
  "gene": "UniProtKB:Q8NGZ4",
  "term_label": "detection of chemical stimulus involved in sensory perception of smell",
  "gene_name": "Olfactory receptor 2G3"
}